cycloartenol synthase activity [GO:0016871] (molecular function) Also known as: oxidosqualene:cycloartenol cyclase activity, (S)-2,3-epoxysqualene mutase (cyclizing, cycloartenol-forming), 2,3-epoxysqualene cycloartenol-cyclase activity, 2,3-epoxysqualene--cycloartenol cyclase activity, 2,3-oxidosqualene-cycloartenol cyclase activity, squalene-2,3-epoxide-cycloartenol cyclase activity Sources: EC:5.4.99.8, RHEA:21308 Definition: Catalysis of the reaction: (S)-2,3-epoxysqualene = cycloartenol. Relationships: is a type of oxidosqualene cyclase activity [GO:0031559]